{
  "gene_symbol": "DYNC2I2",
  "gene_name": "Cytoplasmic dynein 2 intermediate chain 2",
  "term_label": "dynein light chain binding",
  "gene": "UniProtKB:Q96EX3",
  "term_id": "GO:0045503"
}